negative regulation of imaginal disc-derived wing size [GO:0044720] (biological process) Relationships: is a type of regulation of imaginal disc-derived wing size [GO:0044719] Definition: Any process that reduces the size of an imaginal disc-derived wing. References: PMID:21393605